{
  "term_label": "tubulin binding",
  "gene": "UniProtKB:Q9Y238",
  "gene_symbol": "DLEC1",
  "gene_name": "Deleted in lung and esophageal cancer protein 1",
  "term_id": "GO:0015631"
}